{
  "gene_name": "T-box transcription factor TBX19",
  "gene_symbol": "TBX19",
  "term_label": "mesoderm formation",
  "gene": "UniProtKB:O60806",
  "term_id": "GO:0001707"
}